lipooligosaccharide catabolic process [GO:1901270] (biological process) Sources: GOC:TermGenie, GOC:yaf, UniPathway:UPA00501 Also known as: lipooligosaccharide breakdown, lipooligosaccharide catabolism, lipooligosaccharide degradation Definition: The chemical reactions and pathways resulting in the breakdown of lipooligosaccharide. Relationships: is a type of carbohydrate derivative catabolic process [GO:1901136]; is a type of lipooligosaccharide metabolic process [GO:1901269]